positive regulation of protein processing [GO:0010954] (BP) Sources: GOC:dph, GOC:mah, GOC:tb Also known as: positive regulation of protein maturation by peptide bond cleavage Definition: Any process that increases the rate, frequency or extent of protein maturation by peptide bond cleavage. Relationships: is a type of positive regulation of proteolysis [GO:0045862]; is a type of GO:0070613; is a type of GO:1903319; positively regulates protein processing [GO:0016485] Subtypes: Factor XII activation [GO:0002542], GO:0010756, positive regulation of peptide hormone processing [GO:0060569], positive regulation of protein processing in phagocytic vesicle [GO:1903923]